nematode pharynx morphogenesis [GO:0110040] (biological process) Relationships: is a type of animal organ morphogenesis [GO:0009887] Definition: The process in which the anatomical structures of the nematode pharynx are generated and organized. Regulation: regulated by GO:0110041; negatively regulated by GO:0110042; positively regulated by GO:0110043 References: PMID:20805556 Sources: GOC:rz